regulation of adenylate cyclase activity [GO:0045761] (biological process) Subtypes: negative regulation of adenylate cyclase activity [GO:0007194], positive regulation of adenylate cyclase activity [GO:0045762] Also known as: regulation of adenylyl cyclase activity, adenylate cyclase regulator Relationships: is a type of GO:0050790; regulates adenylate cyclase activity [GO:0004016] Definition: Any process that modulates the frequency, rate or extent of adenylate cyclase activity. Sources: GOC:go_curators